{
  "gene": "UniProtKB:Q15075",
  "term_label": "endocytosis",
  "gene_symbol": "EEA1",
  "term_id": "GO:0006897",
  "gene_name": "Early endosome antigen 1"
}